integrin alpha5-beta1 complex [GO:0034674] (cellular component) References: PMID:12297042 Also known as: VLA-5 complex, alpha5-beta1 integrin complex, ITGA5-ITGB1 complex Definition: An integrin complex that comprises one alpha5 subunit and one beta1 subunit. Relationships: is a type of integrin complex [GO:0008305]